{
  "term_label": "RNA polymerase II cis-regulatory region sequence-specific DNA binding",
  "gene": "UniProtKB:P42224",
  "term_id": "GO:0000978",
  "gene_symbol": "STAT1",
  "gene_name": "Signal transducer and activator of transcription 1-alpha_beta"
}